{
  "gene_symbol": "Q5W150",
  "term_id": "UNKNOWN:0003",
  "gene": "UniProtKB:Q5W150",
  "term_label": "Unknown cellular component",
  "gene_name": "Putative uncharacterized protein MGC163334"
}